cellular response to phylloquinone [GO:0071309] (biological process) Also known as: cellular response to vitamin K1 Relationships: is a type of response to phylloquinone [GO:0032573]; is a type of cellular response to vitamin K [GO:0071307] Definition: Any process that results in a change in state or activity of a cell (in terms of movement, secretion, enzyme production, gene expression, etc.) as a result of a phylloquinone (vitamin K1) stimulus. Sources: GOC:mah